{
  "term_id": "GO:0044615",
  "gene_symbol": "NUP35",
  "gene": "UniProtKB:Q8NFH5",
  "gene_name": "Nucleoporin NUP35",
  "term_label": "nuclear pore nuclear basket"
}